{
  "term_id": "GO:0005615",
  "gene": "UniProtKB:O95389",
  "gene_name": "Cellular communication network factor 6",
  "gene_symbol": "CCN6",
  "term_label": "extracellular space"
}